{
  "gene": "UniProtKB:Q6UXH8",
  "gene_name": "Collagen and calcium-binding EGF domain-containing protein 1",
  "gene_symbol": "CCBE1",
  "term_label": "Unknown molecular function",
  "term_id": "UNKNOWN:0001"
}